{
  "gene": "UniProtKB:Q15650",
  "gene_name": "Activating signal cointegrator 1",
  "gene_symbol": "TRIP4",
  "term_id": "GO:0030520",
  "term_label": "estrogen receptor signaling pathway"
}